{
  "gene_symbol": "FHIP2A",
  "term_label": "Unknown cellular component",
  "gene": "UniProtKB:Q5W0V3",
  "term_id": "UNKNOWN:0003",
  "gene_name": "FHF complex subunit HOOK interacting protein 2A"
}